{
  "gene_name": "pre-mRNA 3' end processing protein WDR33",
  "gene": "UniProtKB:Q9C0J8",
  "term_id": "GO:0005847",
  "term_label": "mRNA cleavage and polyadenylation specificity factor complex",
  "gene_symbol": "WDR33"
}